{
  "gene": "UniProtKB:Q86T96",
  "term_id": "GO:0031624",
  "term_label": "ubiquitin conjugating enzyme binding",
  "gene_symbol": "RNF180",
  "gene_name": "E3 ubiquitin-protein ligase RNF180"
}